{
  "gene": "UniProtKB:O75339",
  "gene_symbol": "CILP",
  "gene_name": "Cartilage intermediate layer protein 1",
  "term_id": "GO:0005615",
  "term_label": "extracellular space"
}